{
  "gene_symbol": "TRBV11-2",
  "term_id": "GO:0007166",
  "gene_name": "T cell receptor beta variable 11-2",
  "term_label": "cell surface receptor signaling pathway",
  "gene": "UniProtKB:A0A584"
}